{
  "gene_symbol": "TARS3",
  "term_id": "GO:0004829",
  "gene": "UniProtKB:A2RTX5",
  "term_label": "threonine-tRNA ligase activity",
  "gene_name": "Threonine--tRNA ligase 2, cytoplasmic"
}